{
  "gene": "UniProtKB:Q13643",
  "term_label": "Z disc",
  "gene_symbol": "FHL3",
  "gene_name": "Four and a half LIM domains protein 3",
  "term_id": "GO:0030018"
}